{
  "term_id": "GO:0009566",
  "term_label": "fertilization",
  "gene_name": "Cation channel sperm-associated protein 2",
  "gene_symbol": "CATSPER2",
  "gene": "UniProtKB:Q96P56"
}